{
  "term_label": "cell-cell adhesion mediator activity",
  "gene": "UniProtKB:Q96MS0",
  "term_id": "GO:0098632",
  "gene_symbol": "ROBO3",
  "gene_name": "Roundabout homolog 3"
}